{
  "gene": "UniProtKB:O95863",
  "term_id": "GO:0006355",
  "gene_name": "Zinc finger protein SNAI1",
  "gene_symbol": "SNAI1",
  "term_label": "regulation of DNA-templated transcription"
}